gamma-delta T cell differentiation [GO:0042492] (BP) Subtypes: gamma-delta T cell differentiation involved in immune response [GO:0002303], gamma-delta intraepithelial T cell differentiation [GO:0002304] Note: Note that immunologists typically use the word 'development' to refer to cells of B or T cell lineages undergoing the process that GO describes as 'cell differentiation'. Relationships: is a type of T cell differentiation [GO:0030217]; is a type of GO:0046629 Also known as: gamma-delta T lymphocyte differentiation, gamma-delta T-cell differentiation, gamma-delta T-lymphocyte differentiation, gamma-delta T cell development Regulation: regulated by regulation of gamma-delta T cell differentiation [GO:0045586]; negatively regulated by negative regulation of gamma-delta T cell differentiation [GO:0045587]; positively regulated by positive regulation of gamma-delta T cell differentiation [GO:0045588] Definition: The process in which a relatively unspecialized hemopoietic cell acquires specialized features of a gamma-delta T cell. A gamma-delta T cell is a T cell that expresses a gamma-delta T cell receptor complex. Sources: CL:0000798, GOC:jl